{
  "term_label": "RNA polymerase II cis-regulatory region sequence-specific DNA binding",
  "gene_name": "Zinc finger protein 256",
  "term_id": "GO:0000978",
  "gene_symbol": "ZNF256",
  "gene": "UniProtKB:Q9Y2P7"
}